{
  "term_id": "GO:0003682",
  "term_label": "chromatin binding",
  "gene_symbol": "ACTL6A",
  "gene_name": "Actin-like protein 6A",
  "gene": "UniProtKB:O96019"
}